{
  "term_label": "glycerol metabolic process",
  "gene_name": "Glycerol kinase",
  "gene_symbol": "GK",
  "gene": "UniProtKB:P32189",
  "term_id": "GO:0006071"
}